{
  "term_label": "Unknown molecular function",
  "gene_name": "Proline-rich protein 15-like protein",
  "gene": "UniProtKB:Q9BU68",
  "gene_symbol": "PRR15L",
  "term_id": "UNKNOWN:0001"
}